{
  "gene": "UniProtKB:Q5H9J9",
  "gene_symbol": "TCP11X2",
  "gene_name": "T-complex protein 11 X-linked protein 2",
  "term_id": "GO:0036126",
  "term_label": "sperm flagellum"
}